HU-DNA complex [GO:1990178] (cellular component) Relationships: is a type of protein-DNA complex [GO:0032993]; is a type of GO:1990104; is part of bacterial nucleoid [GO:0043590] Definition: A protein-DNA complex that consists of HU heterodimers (an alpha and a beta chain) assembled into octamers along DNA. HU binds to double-stranded DNA in a structure- and sequence-specific manner and bends the DNA into a nucleosome-like structure. Also known as: HU complex References: PMID:17360520 Sources: GOC:bhm